{
  "term_id": "UNKNOWN:0002",
  "gene_symbol": "SELENBP1",
  "gene_name": "Methanethiol oxidase",
  "gene": "UniProtKB:Q13228",
  "term_label": "Unknown biological process"
}